{
  "term_label": "cytoplasm",
  "gene_name": "Zinc finger CCHC domain-containing protein 3",
  "term_id": "GO:0005737",
  "gene_symbol": "ZCCHC3",
  "gene": "UniProtKB:Q9NUD5"
}